{
  "term_label": "signaling receptor activity",
  "gene": "UniProtKB:P56199",
  "gene_name": "Integrin alpha-1",
  "gene_symbol": "ITGA1",
  "term_id": "GO:0038023"
}